{
  "gene_symbol": "ZNF207",
  "term_id": "GO:0000776",
  "term_label": "kinetochore",
  "gene": "UniProtKB:O43670",
  "gene_name": "BUB3-interacting and GLEBS motif-containing protein ZNF207"
}